sodium-independent organic anion transport [GO:0043252] (biological process) Definition: The directed, sodium-independent, movement of organic anions into, out of or within a cell, or between cells, by means of some agent such as a transporter or pore. Relationships: is a type of GO:0015711 Sources: GOC:go_curators